{
  "term_label": "mitochondrion",
  "gene": "UniProtKB:O75879",
  "gene_symbol": "GATB",
  "gene_name": "Glutamyl-tRNA(Gln) amidotransferase subunit B, mitochondrial",
  "term_id": "GO:0005739"
}